{
  "term_label": "cell surface",
  "gene_name": "Carcinoembryonic antigen-related cell adhesion molecule 4",
  "term_id": "GO:0009986",
  "gene_symbol": "CEACAM4",
  "gene": "UniProtKB:O75871"
}